{
  "term_label": "Unknown cellular component",
  "gene": "UniProtKB:Q9BQA5",
  "gene_name": "Histone H4 transcription factor",
  "term_id": "UNKNOWN:0003",
  "gene_symbol": "HINFP"
}